5'-deoxynucleotidase activity [GO:0002953] (molecular function) Definition: Catalysis of the reaction: a 2'-deoxyribonucleoside 5'-phosphate + H2O = a 2'-deoxyribonucleoside + phosphate. Relationships: is_a phosphatase activity [GO:0016791] Sources: RHEA:36167